peptidoglycan endopeptidase activity [GO:0061785] (molecular function) Subtypes: GO:0061786, GO:0061787 Definition: An endopeptidase activity that uses peptidoglycan as a substrate. References: PMID:22748813 Sources: GOC:dph, GOC:jh Relationships: is a type of endopeptidase activity [GO:0004175]; is a type of peptidoglycan muralytic activity [GO:0061783]